{
  "term_id": "GO:0004074",
  "term_label": "biliverdin reductase [NAD(P)H] activity",
  "gene_symbol": "BLVRB",
  "gene_name": "Flavin reductase (NADPH)",
  "gene": "UniProtKB:P30043"
}